metanephric glomerular epithelial cell development [GO:0072313] (biological process) Subtypes: GO:0072246, GO:0072249 Sources: GOC:mtg_kidney_jan10 Relationships: is a type of GO:0072310; is part of GO:0072312 Definition: The process whose specific outcome is the progression of a metanephric glomerular epithelial cell over time, from its formation to the mature structure. Metanephric glomerular epithelial cells are specialized epithelial cells that form part of the metanephric glomerulus; there are two types, metanephric glomerular parietal epithelial cells and metanephric glomerular visceral epithelial cells.